{
  "gene": "UniProtKB:Q8TCT7",
  "gene_name": "Signal peptide peptidase-like 2B",
  "term_id": "GO:0042500",
  "term_label": "aspartic endopeptidase activity, intramembrane cleaving",
  "gene_symbol": "SPPL2B"
}